{
  "term_label": "establishment or maintenance of cell polarity",
  "term_id": "GO:0007163",
  "gene_name": "Fascin-3",
  "gene": "UniProtKB:Q9NQT6",
  "gene_symbol": "FSCN3"
}